single strand break repair [GO:0000012] (biological process) Definition: The repair of single strand breaks in DNA. Repair of such breaks is mediated by the same enzyme systems as are used in base excision repair. Subtypes: telomere single strand break repair [GO:1903823], GO:1990396 Relationships: is a type of DNA repair [GO:0006281] References: PMID:18626472 Regulation: regulated by regulation of single strand break repair [GO:1903516]; negatively regulated by negative regulation of single strand break repair [GO:1903517]; positively regulated by positive regulation of single strand break repair [GO:1903518]